{
  "gene_symbol": "Q8NFD4",
  "gene": "UniProtKB:Q8NFD4",
  "gene_name": "Uncharacterized protein FLJ76381",
  "term_id": "UNKNOWN:0001",
  "term_label": "Unknown molecular function"
}